{
  "term_label": "peptidyl-prolyl cis-trans isomerase activity",
  "gene": "UniProtKB:Q02790",
  "gene_symbol": "FKBP4",
  "term_id": "GO:0003755",
  "gene_name": "Peptidyl-prolyl cis-trans isomerase FKBP4"
}